{
  "term_label": "nucleus",
  "term_id": "GO:0005634",
  "gene_symbol": "FABP1",
  "gene": "UniProtKB:P07148",
  "gene_name": "Fatty acid-binding protein, liver"
}